endothelin A receptor binding [GO:0031707] (molecular function) Definition: Binding to an endothelin A receptor. Also known as: endothelin-1 receptor binding, endothelin A receptor ligand Sources: GOC:mah, GOC:nln Relationships: is a type of bombesin receptor binding [GO:0031705]